ice nucleation activity [GO:0019833] (molecular function) Note: Note that this term was reinstated from obsolete. Relationships: is a type of ice binding [GO:0050825] References: PMID:35551271 Sources: GOC:cjm, UniProt:KW-0387 Definition: Catalysis of the formation of ice crystals in extracellular fluid at relatively high temperatures (up to -2 degrees Celsius) to protect the organism from damage by intracellular ice formation. This process is commonly found in certain bacteria, such as Pseudomonas syringae, and plays roles in environmental adaptation and plant pathogenesis.